{
  "gene_symbol": "MS4A2",
  "term_label": "cell surface receptor signaling pathway",
  "term_id": "GO:0007166",
  "gene": "UniProtKB:Q01362",
  "gene_name": "High affinity immunoglobulin epsilon receptor subunit beta"
}